{
  "gene_symbol": "RAB12",
  "gene": "UniProtKB:Q6IQ22",
  "gene_name": "Ras-related protein Rab-12",
  "term_id": "GO:0006887",
  "term_label": "exocytosis"
}